mannosome [GO:0042580] (cellular component) Definition: A specialised tubular organelle, assembled in hexagonal bundles within an external membrane. Mannosomes are specific to molluscs and are thought to be involved in a general stress reaction. References: PMID:11912051, PMID:9799531 Sources: GOC:jl Relationships: is_a peroxisome [GO:0005777]